{
  "gene": "UniProtKB:Q9UBQ7",
  "gene_name": "Glyoxylate reductase_hydroxypyruvate reductase",
  "term_label": "glyoxylate reductase (NADPH) activity",
  "term_id": "GO:0030267",
  "gene_symbol": "GRHPR"
}